{
  "gene_name": "Transmembrane protein 94",
  "gene": "UniProtKB:Q12767",
  "term_label": "P-type magnesium transporter activity",
  "term_id": "GO:0015444",
  "gene_symbol": "TMEM94"
}